{
  "gene_symbol": "SOWAHA",
  "gene": "UniProtKB:Q2M3V2",
  "gene_name": "Ankyrin repeat domain-containing protein SOWAHA",
  "term_label": "Unknown biological process",
  "term_id": "UNKNOWN:0002"
}